{
  "gene": "UniProtKB:P17019",
  "gene_name": "Zinc finger protein 708",
  "term_id": "GO:0006355",
  "gene_symbol": "ZNF708",
  "term_label": "regulation of DNA-templated transcription"
}